{
  "gene_name": "Protocadherin alpha-8",
  "gene_symbol": "PCDHA8",
  "term_label": "plasma membrane",
  "term_id": "GO:0005886",
  "gene": "UniProtKB:Q9Y5H6"
}